{
  "gene": "UniProtKB:O95399",
  "gene_symbol": "UTS2",
  "gene_name": "Urotensin-2",
  "term_label": "extracellular space",
  "term_id": "GO:0005615"
}